{
  "term_id": "GO:0032342",
  "term_label": "aldosterone biosynthetic process",
  "gene_symbol": "CYP11B2",
  "gene_name": "Cytochrome P450 11B2, mitochondrial",
  "gene": "UniProtKB:P19099"
}